regulation of translational termination [GO:0006449] (biological process) Sources: GOC:go_curators Relationships: is a type of regulation of translation [GO:0006417]; is a type of regulation of protein-containing complex disassembly [GO:0043244]; regulates translational termination [GO:0006415] Definition: Any process that modulates the frequency, rate or extent of translational termination. Subtypes: GO:0045904, positive regulation of translational termination [GO:0045905], regulation of cytoplasmic translational termination [GO:1990580]